{
  "gene": "UniProtKB:Q8TDY3",
  "term_id": "UNKNOWN:0002",
  "gene_name": "Actin-related protein T2",
  "gene_symbol": "ACTRT2",
  "term_label": "Unknown biological process"
}